{
  "term_id": "GO:0030145",
  "gene_symbol": "SOD2",
  "term_label": "manganese ion binding",
  "gene": "UniProtKB:P04179",
  "gene_name": "Superoxide dismutase [Mn], mitochondrial"
}